{
  "gene": "UniProtKB:A6NGY1",
  "term_label": "Unknown biological process",
  "gene_symbol": "FRG2C",
  "term_id": "UNKNOWN:0002",
  "gene_name": "Protein FRG2-like-2"
}